{
  "gene_name": "Leucine-rich repeat and calponin homology domain-containing protein 1",
  "gene": "UniProtKB:Q9Y2L9",
  "gene_symbol": "LRCH1",
  "term_id": "UNKNOWN:0001",
  "term_label": "Unknown molecular function"
}